G-protein alpha-subunit binding [GO:0001965] (molecular function) Sources: GOC:hjd Also known as: G-alpha protein subunit binding Definition: Binding to a G-protein alpha subunit. The alpha subunit binds a guanine nucleotide. Relationships: is a type of protein binding [GO:0005515]